olfactory bulb mitral cell layer development [GO:0061034] (biological process) Sources: GOC:dph Relationships: is a type of anatomical structure development [GO:0048856]; is part of GO:0021772 Definition: The progression of the olfactory bulb mitral cell layer over time from its initial formation until its mature state. The mitral cell layer is composed of pyramidal neurons whose cell bodies are located between the granule cell layer and the plexiform layer.